{
  "gene_name": "X-ray repair cross-complementing protein 6",
  "term_id": "GO:0000723",
  "term_label": "telomere maintenance",
  "gene": "UniProtKB:P12956",
  "gene_symbol": "XRCC6"
}